{
  "gene_symbol": "LCT",
  "gene_name": "Lactase_phlorizin hydrolase",
  "term_id": "GO:0098591",
  "term_label": "external side of apical plasma membrane",
  "gene": "UniProtKB:P09848"
}